{
  "gene_symbol": "SCML2",
  "gene_name": "Sex comb on midleg-like protein 2",
  "gene": "UniProtKB:Q9UQR0",
  "term_label": "nucleus",
  "term_id": "GO:0005634"
}